{
  "gene_symbol": "SEPTIN6",
  "term_label": "microtubule cytoskeleton",
  "gene_name": "Septin-6",
  "gene": "UniProtKB:Q14141",
  "term_id": "GO:0015630"
}